negative regulation of interleukin-22 production [GO:0032706] (biological process) Definition: Any process that stops, prevents, or reduces the frequency, rate, or extent of interleukin-22 production. Sources: GOC:mah Relationships: is a type of negative regulation of cytokine production [GO:0001818]; is_a GO:0032666; negatively regulates interleukin-22 production [GO:0032626] Also known as: down regulation of interleukin-22 production, down-regulation of interleukin-22 production, downregulation of interleukin-22 production, negative regulation of IL-22 production, inhibition of interleukin-22 production, negative regulation of interleukin-22 biosynthetic process